{
  "gene_symbol": "FOXN3",
  "gene": "UniProtKB:O00409",
  "gene_name": "Forkhead box protein N3",
  "term_id": "GO:0005634",
  "term_label": "nucleus"
}